{
  "term_label": "plasma membrane",
  "gene_name": "Synaptotagmin-like protein 4",
  "gene": "UniProtKB:Q96C24",
  "gene_symbol": "SYTL4",
  "term_id": "GO:0005886"
}